{
  "term_label": "cell chemotaxis",
  "gene_symbol": "CCR10",
  "term_id": "GO:0060326",
  "gene_name": "C-C chemokine receptor type 10",
  "gene": "UniProtKB:P46092"
}